Holliday junction resolvase complex [GO:0048476] (cellular component) Definition: An endodeoxyribonuclease complex that resolves the 4-way DNA intermediates of a Holliday junction into two separate duplex DNA molecules. Can be branch-migration associated. Also known as: resolvasome, Mus81-Eme1 complex, Mus81-Eme1 holliday resolvase complex, Mus81-Eme2 complex, Mus81-Eme2 holliday resolvase complex References: PMID:11207366, PMID:12374758 Relationships: is a type of GO:1905347